{
  "term_label": "cytoplasm",
  "gene_symbol": "TRIM26",
  "term_id": "GO:0005737",
  "gene_name": "Tripartite motif-containing protein 26",
  "gene": "UniProtKB:Q12899"
}